{
  "term_id": "GO:0004571",
  "term_label": "mannosyl-oligosaccharide 1,2-alpha-mannosidase activity",
  "gene": "UniProtKB:Q9NR34",
  "gene_name": "Mannosyl-oligosaccharide 1,2-alpha-mannosidase IC",
  "gene_symbol": "MAN1C1"
}